{
  "term_label": "meiotic cell cycle",
  "gene": "UniProtKB:Q96RT7",
  "gene_name": "Gamma-tubulin complex component 6",
  "gene_symbol": "TUBGCP6",
  "term_id": "GO:0051321"
}